protein localization to cytoskeleton [GO:0044380] (biological process) Relationships: is a type of protein localization to organelle [GO:0033365] Sources: GOC:jl Definition: A process in which a protein is transported to, or maintained in, a location within the cytoskeleton. Subtypes: chromosome passenger complex localization to spindle midzone [GO:0035853], protein localization to microtubule cytoskeleton [GO:0072698], protein localization to eisosome filament [GO:0097446], protein localization to septin ring [GO:1902935], protein localization to actin cytoskeleton [GO:1903119] Also known as: protein localisation to cytoskeleton